thermoception [GO:0050955] (biological process) Subtypes: sensory perception of cold stimulus [GO:0062035], sensory perception of hot stimulus [GO:0062036] Relationships: is a type of GO:0050951 Also known as: thermoreception Sources: GOC:ai, Wikipedia:Thermoception Definition: The series of events required for an organism to receive a temperature stimulus, convert it to a molecular signal, and recognize and characterize the signal. Thermoception in larger animals is mainly done in the skin; mammals have at least two types of sensor, for detecting heat (temperatures above body temperature) and cold (temperatures below body temperature).